anthranilate N-benzoyltransferase activity [GO:0047672] (molecular function) Also known as: benzoyl-CoA:anthranilate N-benzoyltransferase Definition: Catalysis of the reaction: anthranilate + benzoyl-CoA = N-benzoylanthranilate + CoA. Relationships: is a type of acyltransferase activity, transferring groups other than amino-acyl groups [GO:0016747] Sources: EC:2.3.1.144, RHEA:21600